{
  "gene_symbol": "GUF1",
  "term_id": "GO:0045727",
  "term_label": "positive regulation of translation",
  "gene_name": "Translation factor GUF1, mitochondrial",
  "gene": "UniProtKB:Q8N442"
}